{
  "gene": "UniProtKB:Q9C0H9",
  "gene_symbol": "SRCIN1",
  "term_id": "UNKNOWN:0001",
  "term_label": "Unknown molecular function",
  "gene_name": "SRC kinase signaling inhibitor 1"
}